{
  "term_id": "GO:0000045",
  "gene_name": "Ras-related protein Rab-33A",
  "gene_symbol": "RAB33A",
  "gene": "UniProtKB:Q14088",
  "term_label": "autophagosome assembly"
}